{
  "term_label": "Unknown biological process",
  "gene_symbol": "KRTAP9-9",
  "term_id": "UNKNOWN:0002",
  "gene_name": "Keratin-associated protein 9-9",
  "gene": "UniProtKB:Q9BYP9"
}